{
  "gene_symbol": "COMMD6",
  "gene_name": "COMM domain-containing protein 6",
  "term_id": "UNKNOWN:0003",
  "gene": "UniProtKB:Q7Z4G1",
  "term_label": "Unknown cellular component"
}